{
  "gene": "UniProtKB:Q96NG5",
  "gene_name": "Zinc finger protein 558",
  "term_id": "GO:0000981",
  "gene_symbol": "ZNF558",
  "term_label": "DNA-binding transcription factor activity, RNA polymerase II-specific"
}